{
  "gene_name": "Tumor necrosis factor receptor superfamily member 10C",
  "gene": "UniProtKB:O14798",
  "term_label": "positive regulation of apoptotic process",
  "term_id": "GO:0043065",
  "gene_symbol": "TNFRSF10C"
}